{
  "term_label": "animal organ development",
  "term_id": "GO:0048513",
  "gene": "UniProtKB:P51116",
  "gene_name": "RNA-binding protein FXR2",
  "gene_symbol": "FXR2"
}